pathogen-containing vacuole membrane [GO:0140221] (cellular component) Definition: Host-derived membrane of a pathogen-containing vacuole. References: PMID:10560000, PMID:26842840 Also known as: pathogen-containing compartment membrane, pathogen inclusion membrane Relationships: is a type of membrane [GO:0016020]; is part of pathogen-containing vacuole [GO:0140220]